{
  "term_id": "UNKNOWN:0003",
  "term_label": "Unknown cellular component",
  "gene_symbol": "SMCR5",
  "gene": "UniProtKB:Q8TEV8",
  "gene_name": "Smith-Magenis syndrome chromosomal region candidate gene 5 protein"
}